{
  "gene_name": "Pleiotrophin",
  "term_id": "GO:0008083",
  "gene_symbol": "PTN",
  "term_label": "growth factor activity",
  "gene": "UniProtKB:P21246"
}